positive regulation of membrane permeability [GO:1905710] (biological process) Definition: Any process that activates or increases the frequency, rate or extent of the passage or uptake of molecules by a membrane. References: PMID:27482894 Relationships: is a type of regulation of membrane permeability [GO:0090559] Subtypes: positive regulation of mitochondrial membrane permeability [GO:0035794], positive regulation of lysosomal membrane permeability [GO:0097214]